alginic acid biosynthetic process [GO:0042121] (BP) Sources: ISBN:0198506732 Relationships: is a type of polysaccharide biosynthetic process [GO:0000271]; is a type of GO:0046394 Definition: The chemical reactions and pathways resulting in the formation of alginic acid, a hydrophilic polysaccharide occurring in, for example, the cell walls of brown algae (brown seaweeds). Also known as: alginate biosynthesis, alginate biosynthetic process, alginic acid anabolism, alginic acid biosynthesis, alginic acid formation, alginic acid synthesis